{
  "gene_name": "SERTA domain-containing protein 2",
  "gene_symbol": "SERTAD2",
  "gene": "UniProtKB:Q14140",
  "term_label": "transcription coactivator activity",
  "term_id": "GO:0003713"
}